{
  "gene": "UniProtKB:Q15735",
  "term_label": "plasma membrane",
  "term_id": "GO:0005886",
  "gene_name": "Phosphatidylinositol 4,5-bisphosphate 5-phosphatase A",
  "gene_symbol": "INPP5J"
}